{
  "gene": "UniProtKB:Q6AWC2",
  "gene_name": "Protein WWC2",
  "gene_symbol": "WWC2",
  "term_id": "GO:0060090",
  "term_label": "molecular adaptor activity"
}